{
  "gene_symbol": "IL20RA",
  "gene_name": "Interleukin-20 receptor subunit alpha",
  "term_id": "GO:0019221",
  "gene": "UniProtKB:Q9UHF4",
  "term_label": "cytokine-mediated signaling pathway"
}